{
  "gene_name": "Protein MIX23",
  "term_label": "Unknown molecular function",
  "gene_symbol": "MIX23",
  "gene": "UniProtKB:Q4VC31",
  "term_id": "UNKNOWN:0001"
}